{
  "gene": "UniProtKB:Q9NXS3",
  "gene_name": "Kelch-like protein 28",
  "term_label": "cytoplasm",
  "term_id": "GO:0005737",
  "gene_symbol": "KLHL28"
}